{
  "gene_name": "T cell receptor gamma variable 4",
  "term_label": "Unknown biological process",
  "term_id": "UNKNOWN:0002",
  "gene_symbol": "TRGV4",
  "gene": "UniProtKB:A0A0C4DH28"
}